lipoxin A4 biosynthetic process [GO:2001303] (biological process) Definition: The chemical reactions and pathways resulting in the formation of lipoxin A4. Lipoxin A4 is a C20 hydroxy fatty acid having (5S)-, (6R)- and (15S)-hydroxy groups as well as (7E)- (9E)-, (11Z)- and (13E)-double bonds. Sources: GOC:mw Also known as: LXA4 anabolism, LXA4 biosynthesis, LXA4 biosynthetic process, LXA4 formation, LXA4 synthesis, lipoxin A4 anabolism, lipoxin A4 biosynthesis, lipoxin A4 formation, lipoxin A4 synthesis Relationships: is a type of unsaturated fatty acid biosynthetic process [GO:0006636]; is a type of long-chain fatty acid biosynthetic process [GO:0042759]; is a type of lipoxin biosynthetic process [GO:2001301]; is a type of GO:2001302